{
  "term_label": "Unknown cellular component",
  "gene_name": "BEN domain-containing protein 7",
  "term_id": "UNKNOWN:0003",
  "gene": "UniProtKB:Q8N7W2",
  "gene_symbol": "BEND7"
}